{
  "gene": "UniProtKB:Q9H0V9",
  "term_id": "GO:0000139",
  "gene_symbol": "LMAN2L",
  "gene_name": "VIP36-like protein",
  "term_label": "Golgi membrane"
}